{
  "gene_name": "Signal transducer and activator of transcription 3",
  "term_id": "GO:0000978",
  "gene_symbol": "STAT3",
  "gene": "UniProtKB:P40763",
  "term_label": "RNA polymerase II cis-regulatory region sequence-specific DNA binding"
}